{
  "gene_symbol": "PAOX",
  "term_label": "spermidine catabolic process",
  "gene_name": "Peroxisomal N(1)-acetyl-spermine_spermidine oxidase",
  "term_id": "GO:0046203",
  "gene": "UniProtKB:Q6QHF9"
}